{
  "gene": "UniProtKB:A0A0B4J234",
  "gene_name": "T cell receptor alpha variable 2",
  "gene_symbol": "TRAV2",
  "term_id": "GO:0019814",
  "term_label": "immunoglobulin complex"
}